8-oxo-7,8-dihydroguanine DNA N-glycosylase activity [GO:0034039] (molecular function) Relationships: is a type of oxidized purine nucleobase lesion DNA N-glycosylase activity [GO:0008534] References: PMID:17641464 Sources: GOC:mah Definition: Catalysis of the removal of 8-oxo-7,8-dihydroguanine bases by cleaving the N-C1' glycosidic bond between the oxidized purine and the deoxyribose sugar. Also known as: 8-oxoG DNA N-glycosylase activity